adenosine catabolic process [GO:0006154] (biological process) Definition: The chemical reactions and pathways resulting in the breakdown of adenosine, adenine riboside, a ribonucleoside found widely distributed in cells of every type as the free nucleoside and in combination in nucleic acids and various nucleoside coenzymes. Sources: GOC:go_curators Also known as: adenosine breakdown, adenosine catabolism, adenosine degradation, adenosine phosphorolysis Relationships: is_a adenosine metabolic process [GO:0046085]; is a type of GO:0046130